{
  "term_label": "phosphatidylserine binding",
  "term_id": "GO:0001786",
  "gene": "UniProtKB:P07355",
  "gene_symbol": "ANXA2",
  "gene_name": "Annexin A2"
}